telomerase activity [GO:0003720] (molecular function) References: PMID:11812242, PMID:28732250 Sources: GOC:krc Also known as: telomerase RNA reverse transcriptase activity, telomerase, catalyst Definition: Catalysis of the reaction: a 2'-deoxyribonucleoside 5'-triphosphate + DNA(n) = diphosphate + DNA(n+1) using an internal RNA template that encodes the telomeric repeat sequence. Relationships: is a type of RNA-directed DNA polymerase activity [GO:0003964] Regulation: negatively regulated by GO:0010521